structural constituent of vitelline membrane [GO:0008316] (molecular function) Sources: GOC:mah, GOC:sensu Relationships: is a type of structural molecule activity [GO:0005198] Definition: The action of a molecule that contributes to the structural integrity of the vitelline membrane of an egg. An example of this is found in Drosophila melanogaster.